GDP-fucose import into Golgi lumen [GO:0036085] (biological process) Also known as: GDP-fucose import into Golgi, GDP-fucose transport across Golgi membrane, GDP-fucose transport into Golgi lumen Relationships: is a type of GDP-fucose transmembrane transport [GO:0015783]; is a type of GO:0140820 Definition: The directed movement of GDP-fucose into the Golgi lumen. GDP-fucose is a substance composed of fucose in glycosidic linkage with guanosine diphosphate. References: PMID:3458237 Sources: GOC:sart